{
  "term_id": "GO:0045717",
  "gene": "UniProtKB:Q96JK2",
  "gene_symbol": "DCAF5",
  "gene_name": "DDB1- and CUL4-associated factor 5",
  "term_label": "negative regulation of fatty acid biosynthetic process"
}